{
  "term_id": "UNKNOWN:0001",
  "gene": "UniProtKB:Q8N6M6",
  "gene_symbol": "AOPEP",
  "term_label": "Unknown molecular function",
  "gene_name": "Aminopeptidase O"
}